{
  "term_label": "synapse organization",
  "term_id": "GO:0050808",
  "gene": "UniProtKB:Q9BYB0",
  "gene_name": "SH3 and multiple ankyrin repeat domains protein 3",
  "gene_symbol": "SHANK3"
}